aggresome assembly [GO:0070842] (biological process) Definition: The aggregation, arrangement and bonding together of a set of components to form an aggresome; requires the microtubule cytoskeleton and dynein. References: PMID:14675537 Sources: GOC:BHF, GOC:rl Relationships: is a type of inclusion body assembly [GO:0070841]